{
  "term_label": "plasma membrane",
  "gene_symbol": "KLRC3",
  "term_id": "GO:0005886",
  "gene": "UniProtKB:Q07444",
  "gene_name": "NKG2-E type II integral membrane protein"
}